{
  "gene_symbol": "PSMD5",
  "gene_name": "26S proteasome non-ATPase regulatory subunit 5",
  "gene": "UniProtKB:Q16401",
  "term_id": "UNKNOWN:0003",
  "term_label": "Unknown cellular component"
}